small RNA 2'-O-methyltransferase activity [GO:0090486] (MF) Definition: Catalysis of the transfer of a methyl group from S-adenosyl-L-methionine to the oxygen atom of a nucleoside residue in a small RNA molecule. Reaction: S-adenosyl-L-methionine + small RNA = S-adenosyl-L-homocysteine + small RNA containing a 3'-terminal 2'-O-methylnucleotide. Sources: GOC:tb, GOC:vw, RHEA:37887 Subtypes: U6 snRNA 2'-O-ribose methyltransferase activity [GO:0180021] Also known as: small RNA 2'-O-methyltransferase Relationships: is a type of RNA 2'-O-methyltransferase activity [GO:0062105]